histone acetyltransferase binding [GO:0035035] (molecular function) Definition: Binding to an histone acetyltransferase. Also known as: histone acetylase binding Sources: GOC:bf Relationships: is a type of GO:0019899